{
  "gene_symbol": "ACTL8",
  "gene": "UniProtKB:Q9H568",
  "term_id": "GO:0005884",
  "gene_name": "Actin-like protein 8",
  "term_label": "actin filament"
}